{
  "gene": "UniProtKB:Q9P217",
  "term_label": "Unknown biological process",
  "term_id": "UNKNOWN:0002",
  "gene_name": "Zinc finger SWIM domain-containing protein 5",
  "gene_symbol": "ZSWIM5"
}